{
  "term_label": "Unknown molecular function",
  "gene_symbol": "KIAA0408",
  "term_id": "UNKNOWN:0001",
  "gene_name": "Uncharacterized protein KIAA0408",
  "gene": "UniProtKB:Q6ZU52"
}